{
  "term_id": "GO:0016020",
  "gene_name": "Endophilin-A1",
  "gene_symbol": "SH3GL2",
  "term_label": "membrane",
  "gene": "UniProtKB:Q99962"
}